{
  "gene_name": "Small integral membrane protein 34",
  "gene": "UniProtKB:A8MWV9",
  "gene_symbol": "SMIM34",
  "term_id": "UNKNOWN:0001",
  "term_label": "Unknown molecular function"
}